{
  "term_label": "4-alpha-glucanotransferase activity",
  "gene_name": "Glycogen debranching enzyme",
  "gene": "UniProtKB:P35573",
  "gene_symbol": "AGL",
  "term_id": "GO:0004134"
}